{
  "term_id": "GO:0032869",
  "gene_symbol": "LPIN1",
  "gene_name": "Phosphatidate phosphatase LPIN1",
  "term_label": "cellular response to insulin stimulus",
  "gene": "UniProtKB:Q14693"
}